{
  "gene": "UniProtKB:P43080",
  "gene_symbol": "GUCA1A",
  "term_label": "regulation of signal transduction",
  "term_id": "GO:0009966",
  "gene_name": "Guanylyl cyclase-activating protein 1"
}